{
  "term_id": "UNKNOWN:0001",
  "term_label": "Unknown molecular function",
  "gene": "UniProtKB:Q6JVE6",
  "gene_symbol": "LCN10",
  "gene_name": "Epididymal-specific lipocalin-10"
}